{
  "gene_name": "SRR1-like protein",
  "term_id": "UNKNOWN:0002",
  "gene": "UniProtKB:Q9UH36",
  "term_label": "Unknown biological process",
  "gene_symbol": "SRRD"
}